{
  "gene_name": "FERM domain-containing protein 6",
  "term_id": "GO:0035332",
  "gene": "UniProtKB:Q96NE9",
  "term_label": "positive regulation of hippo signaling",
  "gene_symbol": "FRMD6"
}